{
  "gene_name": "Presequence protease, mitochondrial",
  "gene_symbol": "PITRM1",
  "gene": "UniProtKB:Q5JRX3",
  "term_label": "metalloendopeptidase activity",
  "term_id": "GO:0004222"
}